positive regulation of feeding behavior [GO:2000253] (BP) Also known as: positive regulation of behavioral response to food, positive regulation of behavioural response to food, positive regulation of feeding behaviour, positive regulation of drinking, positive regulation of eating Sources: GOC:obol Definition: Any process that activates or increases the frequency, rate or extent of feeding behavior. Relationships: is a type of positive regulation of behavior [GO:0048520]; is a type of regulation of feeding behavior [GO:0060259]; positively regulates GO:0007631 Subtypes: positive regulation of eating behavior [GO:1904000]